{
  "term_id": "GO:0007043",
  "gene": "UniProtKB:P55286",
  "gene_name": "Cadherin-8",
  "gene_symbol": "CDH8",
  "term_label": "cell-cell junction assembly"
}